{
  "gene": "UniProtKB:Q99877",
  "term_label": "innate immune response in mucosa",
  "term_id": "GO:0002227",
  "gene_symbol": "H2BC15",
  "gene_name": "Histone H2B type 1-N"
}